{
  "gene_symbol": "LAMP3",
  "gene": "UniProtKB:Q9UQV4",
  "term_id": "GO:0072594",
  "gene_name": "Lysosome-associated membrane glycoprotein 3",
  "term_label": "establishment of protein localization to organelle"
}